{
  "gene": "UniProtKB:Q15493",
  "term_label": "gluconolactonase activity",
  "gene_name": "Regucalcin",
  "term_id": "GO:0004341",
  "gene_symbol": "RGN"
}